{
  "gene_name": "Cyclic AMP-dependent transcription factor ATF-4",
  "gene": "UniProtKB:P18848",
  "gene_symbol": "ATF4",
  "term_id": "GO:0000977",
  "term_label": "RNA polymerase II transcription regulatory region sequence-specific DNA binding"
}